phage shock [GO:0009271] (biological process) Definition: A response by bacterial cells to a variety of stresses including filamentous phage infection, mislocalization of envelope proteins, extremes of temperature, osmolarity or ethanol concentration, and the presence of proton ionophores such as carbonylcyanide m-chlorophenylhydrazone (CCCP), that involves expression of the phage shock protein operon, and acts to protect the bacterial cells from damage. References: PMID:15485810, PMID:16045608 Sources: GOC:add, GOC:jl Relationships: is a type of response to stress [GO:0006950]